regulation of gamma-delta T cell activation involved in immune response [GO:2001191] (biological process) Also known as: regulation of gamma-delta T cell activation during immune response, regulation of gamma-delta T lymphocyte activation during immune response, regulation of gamma-delta T-cell activation during immune response, regulation of gamma-delta T-lymphocyte activation during immune response Subtypes: negative regulation of gamma-delta T cell activation involved in immune response [GO:2001192], positive regulation of gamma-delta T cell activation involved in immune response [GO:2001193] Relationships: is a type of GO:0002697; is a type of regulation of gamma-delta T cell activation [GO:0046643]; is a type of regulation of immune response [GO:0050776]; regulates gamma-delta T cell activation involved in immune response [GO:0002290] Sources: GOC:obol Definition: Any process that modulates the frequency, rate or extent of gamma-delta T cell activation involved in immune response.